{
  "term_label": "platelet-derived growth factor receptor binding",
  "gene_symbol": "PDGFC",
  "gene_name": "Platelet-derived growth factor C",
  "gene": "UniProtKB:Q9NRA1",
  "term_id": "GO:0005161"
}